{
  "gene": "UniProtKB:A4FU49",
  "term_id": "UNKNOWN:0003",
  "gene_name": "SH3 domain-containing protein 21",
  "term_label": "Unknown cellular component",
  "gene_symbol": "SH3D21"
}